positive regulation of activated CD8-positive, alpha-beta T cell apoptotic process [GO:1905404] (biological process) Relationships: is a type of positive regulation of T cell apoptotic process [GO:0070234]; is a type of GO:1905402; RO_0002213 activated CD8-positive, alpha-beta T cell apoptotic process [GO:1905397] References: PMID:24187568 Sources: GOC:TermGenie, GO_REF:0000058 Definition: Any process that activates or increases the frequency, rate or extent of activated CD8-positive, alpha-beta T cell apoptotic process. Also known as: positive regulation of activated CD8-positive, alpha-beta T lymphocyte apoptotic process, positive regulation of activated CD8-positive, alpha-beta T-cell apoptotic process, positive regulation of activated CD8-positive, alpha-beta T-lymphocyte apoptotic process, up regulation of activated CD8-positive, alpha-beta T cell apoptotic process, up regulation of activated CD8-positive, alpha-beta T lymphocyte apoptotic process, up regulation of activated CD8-positive, alpha-beta T-cell apoptotic process, up regulation of activated CD8-positive, alpha-beta T-lymphocyte apoptotic process, up-regulation of activated CD8-positive, alpha-beta T cell apoptotic process, up-regulation of activated CD8-positive, alpha-beta T lymphocyte apoptotic process, up-regulation of activated CD8-positive, alpha-beta T-cell apoptotic process, up-regulation of activated CD8-positive, alpha-beta T-lymphocyte apoptotic process, upregulation of activated CD8-positive, alpha-beta T cell apoptotic process, upregulation of activated CD8-positive, alpha-beta T lymphocyte apoptotic process, upregulation of activated CD8-positive, alpha-beta T-cell apoptotic process, upregulation of activated CD8-positive, alpha-beta T-lymphocyte apoptotic process, activation of activated CD8-positive, alpha-beta T cell apoptosis, activation of activated CD8-positive, alpha-beta T cell apoptotic process, activation of activated CD8-positive, alpha-beta T lymphocyte apoptosis, activation of activated CD8-positive, alpha-beta T lymphocyte apoptotic process, activation of activated CD8-positive, alpha-beta T-cell apoptosis, activation of activated CD8-positive, alpha-beta T-cell apoptotic process, activation of activated CD8-positive, alpha-beta T-lymphocyte apoptosis, activation of activated CD8-positive, alpha-beta T-lymphocyte apoptotic process, positive regulation of activated CD8-positive, alpha-beta T cell apoptosis, positive regulation of activated CD8-positive, alpha-beta T lymphocyte apoptosis, positive regulation of activated CD8-positive, alpha-beta T-cell apoptosis, positive regulation of activated CD8-positive, alpha-beta T-lymphocyte apoptosis, up regulation of activated CD8-positive, alpha-beta T cell apoptosis, up regulation of activated CD8-positive, alpha-beta T lymphocyte apoptosis, up regulation of activated CD8-positive, alpha-beta T-cell apoptosis, up regulation of activated CD8-positive, alpha-beta T-lymphocyte apoptosis, up-regulation of activated CD8-positive, alpha-beta T cell apoptosis, up-regulation of activated CD8-positive, alpha-beta T lymphocyte apoptosis, up-regulation of activated CD8-positive, alpha-beta T-cell apoptosis, up-regulation of activated CD8-positive, alpha-beta T-lymphocyte apoptosis, upregulation of activated CD8-positive, alpha-beta T cell apoptosis, upregulation of activated CD8-positive, alpha-beta T lymphocyte apoptosis, upregulation of activated CD8-positive, alpha-beta T-cell apoptosis, upregulation of activated CD8-positive, alpha-beta T-lymphocyte apoptosis